{
  "gene": "UniProtKB:P35462",
  "term_id": "GO:0014059",
  "term_label": "regulation of dopamine secretion",
  "gene_symbol": "DRD3",
  "gene_name": "D(3) dopamine receptor"
}